{
  "term_id": "GO:0005739",
  "gene_name": "WD repeat-containing protein 81",
  "gene_symbol": "WDR81",
  "term_label": "mitochondrion",
  "gene": "UniProtKB:Q562E7"
}